{
  "gene_symbol": "TCIRG1",
  "gene_name": "V-type proton ATPase 116 kDa subunit a 3",
  "term_label": "vacuolar proton-transporting V-type ATPase complex",
  "gene": "UniProtKB:Q13488",
  "term_id": "GO:0016471"
}